{
  "gene": "UniProtKB:Q14573",
  "term_label": "plasma membrane",
  "gene_symbol": "ITPR3",
  "gene_name": "Inositol 1,4,5-trisphosphate receptor type 3",
  "term_id": "GO:0005886"
}